{
  "gene_symbol": "TIMELESS",
  "term_id": "GO:0006281",
  "gene_name": "Protein timeless homolog",
  "term_label": "DNA repair",
  "gene": "UniProtKB:Q9UNS1"
}